{
  "gene": "UniProtKB:Q9C0F0",
  "gene_symbol": "ASXL3",
  "gene_name": "Putative Polycomb group protein ASXL3",
  "term_id": "GO:0035517",
  "term_label": "PR-DUB complex"
}